{
  "gene": "UniProtKB:Q8IVF6",
  "gene_symbol": "ANKRD18A",
  "gene_name": "Ankyrin repeat domain-containing protein 18A",
  "term_label": "Unknown biological process",
  "term_id": "UNKNOWN:0002"
}